{
  "gene_symbol": "MUC5B",
  "gene": "UniProtKB:Q9HC84",
  "gene_name": "Mucin-5B",
  "term_label": "Unknown biological process",
  "term_id": "UNKNOWN:0002"
}